hydrolase activity [GO:0016787] (molecular function) Regulation: regulated by regulation of hydrolase activity [GO:0051336]; RO_0002213 by positive regulation of hydrolase activity [GO:0051345]; negatively regulated by negative regulation of hydrolase activity [GO:0051346] Relationships: is_a catalytic activity [GO:0003824] Definition: Catalysis of the hydrolysis of various bonds, e.g. C-O, C-N, C-C, phosphoric anhydride bonds, etc. Subtypes: peptidase activity [GO:0008233], hydrolase activity, acting on ester bonds [GO:0016788], hydrolase activity, acting on glycosyl bonds [GO:0016798], hydrolase activity, acting on ether bonds [GO:0016801], hydrolase activity, acting on carbon-nitrogen (but not peptide) bonds [GO:0016810], hydrolase activity, acting on acid anhydrides [GO:0016817], hydrolase activity, acting on acid carbon-carbon bonds [GO:0016822], hydrolase activity, acting on acid halide bonds [GO:0016824], hydrolase activity, acting on acid phosphorus-nitrogen bonds [GO:0016825], hydrolase activity, acting on acid sulfur-nitrogen bonds [GO:0016826], GO:0016827, GO:0016828, serine hydrolase activity [GO:0017171], protein-phosphatidylethanolamide deconjugating activity [GO:0019786], steryl deacetylase activity [GO:0034084], hydrolase activity, acting on carbon-sulfur bonds [GO:0046508], cytosine C-5 DNA demethylase activity [GO:0051747], GO:0098599 Sources: ISBN:0198506732